{
  "term_id": "GO:0000139",
  "term_label": "Golgi membrane",
  "gene_symbol": "MAN2A2",
  "gene_name": "Alpha-mannosidase 2x",
  "gene": "UniProtKB:P49641"
}